macrophage migration inhibitory factor production [GO:0044807] (BP) Definition: The appearance of macrophage migration inhibitory factor due to biosynthesis or secretion following a cellular stimulus, resulting in an increase in its intracellular or extracellular levels. Also known as: MIF production Relationships: is a type of cytokine production [GO:0001816] Sources: GOC:rv